{
  "gene_name": "Putative uncharacterized protein LOC642776",
  "term_id": "UNKNOWN:0001",
  "gene": "UniProtKB:Q9BTK2",
  "term_label": "Unknown molecular function",
  "gene_symbol": "Q9BTK2"
}